{
  "gene_symbol": "MYH7",
  "term_id": "GO:0032982",
  "gene": "UniProtKB:P12883",
  "gene_name": "Myosin-7",
  "term_label": "myosin filament"
}